{
  "term_id": "GO:0006833",
  "gene": "UniProtKB:O75631",
  "term_label": "water transport",
  "gene_symbol": "UPK3A",
  "gene_name": "Uroplakin-3a"
}